{
  "gene": "UniProtKB:Q13563",
  "term_label": "muscle alpha-actinin binding",
  "term_id": "GO:0051371",
  "gene_name": "Polycystin-2",
  "gene_symbol": "PKD2"
}